{
  "gene_symbol": "ACTR2",
  "term_label": "actin filament binding",
  "gene_name": "Actin-related protein 2",
  "term_id": "GO:0051015",
  "gene": "UniProtKB:P61160"
}